{
  "gene_symbol": "KCNK1",
  "term_label": "plasma membrane",
  "gene": "UniProtKB:O00180",
  "term_id": "GO:0005886",
  "gene_name": "Potassium channel subfamily K member 1"
}